{
  "term_label": "apical plasma membrane",
  "gene_symbol": "OCEL1",
  "gene_name": "Occludin_ELL domain-containing protein 1",
  "gene": "UniProtKB:Q9H607",
  "term_id": "GO:0016324"
}